{
  "term_id": "UNKNOWN:0002",
  "gene": "UniProtKB:Q9GZU5",
  "gene_symbol": "NYX",
  "term_label": "Unknown biological process",
  "gene_name": "Nyctalopin"
}